C2 axonemal microtubule [GO:1990720] (cellular component) Definition: One of two microtubules present in the axonemal central pair. It is distinguishable from the C1 axonemal microtubule (also called C1 tubule) by the presence of differing protein components of the projections. References: PMID:21586547, PMID:9295136 Sources: GOC:cilia Also known as: C2 tubule Relationships: is a type of axonemal microtubule [GO:0005879]; is part of axonemal central pair [GO:0097540]